response to amino acid starvation [GO:1990928] (biological process) Relationships: is a type of response to starvation [GO:0042594] References: PMID:7765311 Subtypes: cellular response to amino acid starvation [GO:0034198] Definition: Any process that results in a change in state or activity of a cell or an organism (in terms of movement, secretion, enzyme production, gene expression, etc.) as a result of deprivation of amino acids.